TORC2 complex [GO:0031932] (cellular component) Relationships: is a type of TOR complex [GO:0038201] Definition: A protein complex that contains at least TOR (target of rapamycin) and Rictor (rapamycin-insensitive companion of TOR), or orthologs of, in complex with other signaling components. Mediates the phosphorylation and activation of PKB (also called AKT). In Saccharomyces, the complex contains Avo1p, Avo2p, Tsc11p, Lst8p, Bit61p, Slm1p, Slm2p, and Tor2p. References: PMID:14736892, PMID:15780592, PMID:16469695, PMID:21548787 Sources: GOC:bf, GOC:jh Also known as: TOR complex 2, TORC 2 complex, TORC2, rapamycin and nutrient-insensitive TOR complex, mTORC2